{
  "gene_name": "Serine protease inhibitor Kazal-type 5",
  "gene_symbol": "SPINK5",
  "term_label": "serine-type endopeptidase inhibitor activity",
  "gene": "UniProtKB:Q9NQ38",
  "term_id": "GO:0004867"
}